{
  "gene_symbol": "SYT3",
  "term_id": "GO:0016192",
  "gene_name": "Synaptotagmin-3",
  "gene": "UniProtKB:Q9BQG1",
  "term_label": "vesicle-mediated transport"
}